cisternal progression [GO:0045057] (biological process) Sources: ISBN:0716731363 Also known as: cisternal maturation Relationships: is a type of intra-Golgi vesicle-mediated transport [GO:0006891] Definition: The process that results in the physical movement of a new cis-Golgi stack from the cis-position, nearest the endoplasmic reticulum (ER), to the trans position, farthest from the ER, successively becoming first a medial-Golgi cisterna and then a trans-Golgi cisterna.